{
  "gene_symbol": "DEFB131B",
  "term_label": "extracellular space",
  "gene_name": "Beta-defensin 131B",
  "term_id": "GO:0005615",
  "gene": "UniProtKB:A0A096LNP1"
}